platelet alpha granule lumen [GO:0031093] (cellular component) Relationships: is a type of secretory granule lumen [GO:0034774]; is part of platelet alpha granule [GO:0031091] Also known as: platelet alpha-granule lumen Definition: The volume enclosed by the membrane of the platelet alpha granule. References: PMID:8467233 Sources: GOC:mah